{
  "term_id": "GO:0005886",
  "gene_symbol": "RET",
  "term_label": "plasma membrane",
  "gene": "UniProtKB:P07949",
  "gene_name": "Proto-oncogene tyrosine-protein kinase receptor Ret"
}